{
  "gene_symbol": "UQCC5",
  "term_id": "UNKNOWN:0002",
  "gene": "UniProtKB:Q8WVI0",
  "gene_name": "Ubiquinol-cytochrome-c reductase complex assembly factor 5",
  "term_label": "Unknown biological process"
}